{
  "gene_name": "Intestinal-type alkaline phosphatase",
  "term_id": "GO:0005886",
  "gene": "UniProtKB:P09923",
  "term_label": "plasma membrane",
  "gene_symbol": "ALPI"
}